{
  "term_label": "regulation of Rab protein signal transduction",
  "gene_symbol": "DENND3",
  "gene": "UniProtKB:A2RUS2",
  "gene_name": "DENN domain-containing protein 3",
  "term_id": "GO:0032483"
}